{
  "term_label": "histone acetyltransferase complex",
  "gene_symbol": "EP300",
  "term_id": "GO:0000123",
  "gene": "UniProtKB:Q09472",
  "gene_name": "Histone acetyltransferase p300"
}